negative regulation of calcium ion import into sarcoplasmic reticulum [GO:1902081] (biological process) Definition: Any process that stops, prevents or reduces the frequency, rate or extent of calcium ion import into sarcoplasmic reticulum. References: PMID:8349590 Sources: GOC:BHF, GOC:TermGenie, GOC:rl Relationships: is a type of GO:0032387; is a type of negative regulation of calcium ion transport [GO:0051926]; is a type of regulation of calcium ion import into sarcoplasmic reticulum [GO:1902080]; negatively regulates calcium ion import into sarcoplasmic reticulum [GO:1990036] Also known as: down regulation of calcium ion import into sarcoplasmic reticulum, down-regulation of calcium ion import into sarcoplasmic reticulum, downregulation of calcium ion import into sarcoplasmic reticulum, inhibition of calcium ion import into sarcoplasmic reticulum